{
  "gene_symbol": "ETHE1",
  "gene": "UniProtKB:O95571",
  "term_label": "mitochondrion",
  "term_id": "GO:0005739",
  "gene_name": "Persulfide dioxygenase ETHE1, mitochondrial"
}